positive regulation of ATP metabolic process [GO:1903580] (biological process) Relationships: is a type of positive regulation of purine nucleotide metabolic process [GO:1900544]; is a type of regulation of ATP metabolic process [GO:1903578]; RO_0002213 GO:0046034 Definition: Any process that activates or increases the frequency, rate or extent of ATP metabolic process. Subtypes: positive regulation of glycolytic process [GO:0045821], GO:2001171 Also known as: positive regulation of ATP metabolism, up regulation of ATP metabolic process, up regulation of ATP metabolism, up-regulation of ATP metabolic process, up-regulation of ATP metabolism, upregulation of ATP metabolic process, upregulation of ATP metabolism, activation of ATP metabolic process, activation of ATP metabolism References: PMID:20695849 Sources: GOC:TermGenie, GO_REF:0000058